{
  "gene_symbol": "SENP7",
  "term_label": "SUMO-specific endopeptidase activity",
  "term_id": "GO:0070139",
  "gene": "UniProtKB:Q9BQF6",
  "gene_name": "Sentrin-specific protease 7"
}